amine N-methyltransferase activity [GO:0030748] (molecular function) Also known as: arylamine N-methyltransferase activity, nicotine N-methyltransferase activity, tryptamine N-methyltransferase activity, tryptamine methyltransferase, S-adenosyl-L-methionine:amine N-methyltransferase activity Relationships: is_a S-adenosylmethionine-dependent methyltransferase activity [GO:0008757] Sources: EC:2.1.1.49 Definition: Catalysis of the reaction: S-adenosyl-L-methionine + an amine = S-adenosyl-L-homocysteine + a methylated amine. Acts on primary, secondary and tertiary amines.